{
  "term_id": "GO:0006744",
  "gene": "UniProtKB:Q9Y5Z9",
  "gene_symbol": "UBIAD1",
  "term_label": "ubiquinone biosynthetic process",
  "gene_name": "UbiA prenyltransferase domain-containing protein 1"
}